{
  "gene_name": "Transcription initiation factor TFIID subunit 10",
  "gene": "UniProtKB:Q12962",
  "gene_symbol": "TAF10",
  "term_label": "transcription factor TFIID complex",
  "term_id": "GO:0005669"
}